{
  "gene_symbol": "PGR",
  "term_id": "GO:0005634",
  "gene": "UniProtKB:P06401",
  "term_label": "nucleus",
  "gene_name": "Progesterone receptor"
}